{
  "term_id": "UNKNOWN:0002",
  "gene_name": "Prickle-like protein 1",
  "gene_symbol": "PRICKLE1",
  "term_label": "Unknown biological process",
  "gene": "UniProtKB:Q96MT3"
}